acrosome matrix dispersal [GO:0002077] (biological process) Relationships: is a type of proteolysis involved in protein catabolic process [GO:0051603]; is part of acrosome reaction [GO:0007340] References: PMID:3886029 Sources: GOC:dph Definition: The proteolytic digestion of components in the acrosomal matrix that occurs as part of the acrosome reaction. The process can occur either in the cumulus oophorous facilitating the penetration of it by the sperm, or at the zona pellucida allowing the sperm to reach the plasma membrane of the egg where the inner acrosomal membrane of the sperm can interact with the egg plasma membrane.